{
  "gene": "UniProtKB:Q8N5W8",
  "term_id": "UNKNOWN:0001",
  "gene_name": "Protein FAM24B",
  "term_label": "Unknown molecular function",
  "gene_symbol": "FAM24B"
}